{
  "term_label": "Unknown molecular function",
  "term_id": "UNKNOWN:0001",
  "gene_symbol": "CFAP251",
  "gene_name": "Cilia- and flagella-associated protein 251",
  "gene": "UniProtKB:Q8TBY9"
}